serine-type peptidase activity [GO:0008236] (molecular function) Also known as: serine protease activity Definition: Catalysis of the hydrolysis of peptide bonds in a polypeptide chain by a catalytic mechanism that involves a catalytic triad consisting of a serine nucleophile that is activated by a proton relay involving an acidic residue (e.g. aspartate or glutamate) and a basic residue (usually histidine). Sources: https://www.ebi.ac.uk/merops/about/glossary.shtml#CATTYPE Regulation: negatively regulated by negative regulation of serine-type peptidase activity [GO:1902572] Relationships: is a type of GO:0008233; is_a serine hydrolase activity [GO:0017171] Subtypes: GO:0004252, serine-type exopeptidase activity [GO:0070008]